{
  "term_id": "GO:0045296",
  "gene": "UniProtKB:Q12864",
  "term_label": "cadherin binding",
  "gene_symbol": "CDH17",
  "gene_name": "Cadherin-17"
}